nuclear receptor-mediated steroid hormone signaling pathway [GO:0030518] (biological process) Relationships: is a type of GO:0043401; is a type of nuclear receptor-mediated signaling pathway [GO:0141193] Also known as: steroid hormone receptor signaling pathway, steroid hormone receptor signalling pathway, intracellular steroid hormone receptor signaling pathway Subtypes: GO:0030520, GO:0030521, nuclear receptor-mediated corticosteroid signaling pathway [GO:0031958], GO:0035076, progesterone receptor signaling pathway [GO:0050847], oxysterol receptor signaling pathway [GO:0141209] Regulation: regulated by GO:0033143; negatively regulated by negative regulation of intracellular steroid hormone receptor signaling pathway [GO:0033144]; positively regulated by positive regulation of intracellular steroid hormone receptor signaling pathway [GO:0033145] Sources: GOC:mah, GOC:signaling Definition: A nuclear receptor-mediated signaling pathway initiated by a steroid binding to an intracellular receptor of the nuclear receptor protein family, and ending with regulation of a downstream cellular process, e.g. transcription.